{
  "term_label": "regulation of T cell cytokine production",
  "gene_symbol": "TNFRSF1B",
  "gene": "UniProtKB:P20333",
  "gene_name": "Tumor necrosis factor receptor superfamily member 1B",
  "term_id": "GO:0002724"
}